metallodipeptidase activity [GO:0070573] (molecular function) Definition: Catalysis of the hydrolysis of a dipeptide by a mechanism in which water acts as a nucleophile, one or two metal ions hold the water molecule in place, and charged amino acid side chains are ligands for the metal ions. Sources: GOC:mah, https://www.ebi.ac.uk/merops/about/glossary.shtml#CATTYPE Also known as: metallo-exo-dipeptidase activity, metalloexodipeptidase activity Relationships: is a type of GO:0008235; is a type of dipeptidase activity [GO:0016805]